{
  "term_id": "GO:0098978",
  "term_label": "glutamatergic synapse",
  "gene_name": "Leucine-rich repeat and fibronectin type-III domain-containing protein 4",
  "gene_symbol": "LRFN4",
  "gene": "UniProtKB:Q6PJG9"
}